late recombination nodule [GO:0005715] (cellular component) Relationships: is a type of GO:0005713 Sources: GOC:elh Definition: An electron dense structure that is associated with meiotic chromosomes in pachytene during meiosis I.